Golgi apparatus subcompartment [GO:0098791] (cellular component) Also known as: Golgi subcompartment Sources: GOC:dos Subtypes: Golgi stack [GO:0005795], trans-Golgi network [GO:0005802], Golgi cisterna [GO:0031985] Definition: A compartment that consists of a lumen and an enclosing membrane, and is part of the Golgi apparatus. Relationships: is a type of organelle subcompartment [GO:0031984]; is part of Golgi apparatus [GO:0005794]